negative regulation of nitrogen cycle metabolic process [GO:1903315] (biological process) Sources: GOC:TermGenie, GOC:vw, GO_REF:0000058 Definition: Any process that stops, prevents or reduces the frequency, rate or extent of nitrogen cycle metabolic process. Subtypes: GO:1901713 Also known as: down regulation of nitrogen cycle metabolic process, down-regulation of nitrogen cycle metabolic process, downregulation of nitrogen cycle metabolic process, inhibition of nitrogen cycle metabolic process Relationships: is a type of negative regulation of metabolic process [GO:0009892]; is a type of regulation of nitrogen cycle metabolic process [GO:1903314]; negatively regulates nitrogen cycle metabolic process [GO:0071941]